{
  "gene_symbol": "TNIP3",
  "gene": "UniProtKB:Q96KP6",
  "gene_name": "TNFAIP3-interacting protein 3",
  "term_label": "Unknown molecular function",
  "term_id": "UNKNOWN:0001"
}